regulation of endothelial cell migration [GO:0010594] (biological process) Definition: Any process that modulates the rate, frequency, or extent of the orderly movement of an endothelial cell into the extracellular matrix to form an endothelium. Sources: GOC:BHF, GOC:dph, GOC:tb Relationships: is a type of regulation of cell migration [GO:0030334]; RO_0002211 endothelial cell migration [GO:0043542] Subtypes: positive regulation of endothelial cell migration [GO:0010595], negative regulation of endothelial cell migration [GO:0010596], regulation of blood vessel endothelial cell migration [GO:0043535], GO:2001026